{
  "gene_name": "AF4_FMR2 family member 4",
  "gene_symbol": "AFF4",
  "term_label": "regulation of DNA-templated transcription",
  "gene": "UniProtKB:Q9UHB7",
  "term_id": "GO:0006355"
}